{
  "gene_name": "Melanocortin receptor 4",
  "term_id": "GO:0060259",
  "term_label": "regulation of feeding behavior",
  "gene": "UniProtKB:P32245",
  "gene_symbol": "MC4R"
}